{
  "gene_name": "Structural maintenance of chromosomes protein 1A",
  "term_id": "GO:0005634",
  "gene": "UniProtKB:Q14683",
  "term_label": "nucleus",
  "gene_symbol": "SMC1A"
}